{
  "gene": "UniProtKB:P50281",
  "gene_name": "Matrix metalloproteinase-14",
  "term_label": "extracellular matrix organization",
  "term_id": "GO:0030198",
  "gene_symbol": "MMP14"
}